{
  "gene": "UniProtKB:Q9H0B8",
  "term_label": "face morphogenesis",
  "gene_symbol": "CRISPLD2",
  "term_id": "GO:0060325",
  "gene_name": "Cysteine-rich secretory protein LCCL domain-containing 2"
}